{
  "term_label": "mitochondrial matrix",
  "term_id": "GO:0005759",
  "gene": "UniProtKB:Q9UIJ7",
  "gene_name": "GTP:AMP phosphotransferase AK3, mitochondrial",
  "gene_symbol": "AK3"
}